dorsolateral trunk neural crest cell migration [GO:0036485] (biological process) Relationships: is a type of GO:0036484 References: PMID:2387238 Sources: GOC:PARL, GOC:bf, GOC:mat Definition: The movement of trunk neural crest cells from the neural tube, travelling dorso-laterally into the ectoderm and continuing toward the ventral midline of the belly. These migrating trunk neural crest cells become melanocytes, the melanin-forming pigment cells. Also known as: dorsolateral trunk NCC migration